regulation of neuron differentiation [GO:0045664] (biological process) Sources: GOC:go_curators Relationships: is a type of regulation of cell differentiation [GO:0045595]; regulates neuron differentiation [GO:0030182] Definition: Any process that modulates the frequency, rate or extent of neuron differentiation. Subtypes: regulation of neuron maturation [GO:0014041], regulation of mechanoreceptor differentiation [GO:0045631], GO:0045665, positive regulation of neuron differentiation [GO:0045666], regulation of photoreceptor cell differentiation [GO:0046532], regulation of timing of neuron differentiation [GO:0060164], regulation of stomach neuroendocrine cell differentiation [GO:0061105], regulation of glutamatergic neuron differentiation [GO:0120006], regulation of spinal cord association neuron differentiation [GO:1902829], regulation of amacrine cell differentiation [GO:1902869], GO:1904338, regulation of cerebellar neuron development [GO:1905079], regulation of forebrain neuron differentiation [GO:2000977]